{
  "gene_name": "Neuroligin-3",
  "gene": "UniProtKB:Q9NZ94",
  "term_id": "GO:0045202",
  "gene_symbol": "NLGN3",
  "term_label": "synapse"
}